{
  "term_id": "UNKNOWN:0002",
  "gene_name": "Membrane-associated phosphatidylinositol transfer protein 3",
  "gene_symbol": "PITPNM3",
  "gene": "UniProtKB:Q9BZ71",
  "term_label": "Unknown biological process"
}